negative regulation of monocyte chemotactic protein-1 production [GO:0071638] (BP) Sources: GOC:mah Relationships: is a type of negative regulation of chemokine production [GO:0032682]; is a type of regulation of monocyte chemotactic protein-1 production [GO:0071637]; negatively regulates monocyte chemotactic protein-1 production [GO:0071605] Also known as: negative regulation of CCL2 production, negative regulation of MCP-1 production Definition: Any process that stops, prevents, or reduces the frequency, rate, or extent of production of monocyte chemotactic protein-1.